{
  "gene_name": "Serine protease 53",
  "gene_symbol": "PRSS53",
  "term_label": "Unknown cellular component",
  "gene": "UniProtKB:Q2L4Q9",
  "term_id": "UNKNOWN:0003"
}